positive regulation of regulation of ascospore wall (1->3)-beta-D-glucan biosynthetic process [GO:0140748] (biological process) Relationships: is a type of regulation of ascospore wall (1->3)-beta-D-glucan biosynthetic process [GO:0060624]; is a type of positive regulation of (1->3)-beta-D-glucan biosynthetic process [GO:0060635]; is_a positive regulation of cell cycle process [GO:0090068]; is a type of positive regulation of reproductive process [GO:2000243]; RO_0002213 ascospore wall (1->3)-beta-D-glucan biosynthetic process [GO:0034413] Definition: Any process that activates or increases the frequency, rate or extent of ascospore wall (1->3)-beta-D-glucan biosynthetic process. References: PMID:19189958